{
  "gene": "UniProtKB:A6NLJ0",
  "gene_symbol": "C2CD4B",
  "term_label": "Unknown biological process",
  "gene_name": "C2 calcium-dependent domain-containing protein 4B",
  "term_id": "UNKNOWN:0002"
}